{
  "term_label": "Unknown molecular function",
  "gene": "UniProtKB:Q9H8U3",
  "term_id": "UNKNOWN:0001",
  "gene_symbol": "ZFAND3",
  "gene_name": "AN1-type zinc finger protein 3"
}